{
  "term_label": "positive regulation of protein secretion",
  "gene_name": "Insulin",
  "gene_symbol": "INS",
  "term_id": "GO:0050714",
  "gene": "UniProtKB:P01308"
}